eye photoreceptor cell differentiation [GO:0001754] (biological process) Relationships: is a type of photoreceptor cell differentiation [GO:0046530]; is part of eye morphogenesis [GO:0048592] Definition: The process in which a relatively unspecialized cell acquires the specialized features of a photoreceptor cell, as found in the eye, the primary visual organ of most organisms. Subtypes: compound eye photoreceptor cell differentiation [GO:0001751], camera-type eye photoreceptor cell differentiation [GO:0060219] Sources: GOC:go_curators